{
  "gene_symbol": "WTIP",
  "term_id": "GO:0005667",
  "gene_name": "Wilms tumor protein 1-interacting protein",
  "gene": "UniProtKB:A6NIX2",
  "term_label": "transcription regulator complex"
}